regulation of type II hypersensitivity [GO:0002892] (biological process) Definition: Any process that modulates the frequency, rate, or extent of type II hypersensitivity. Sources: GOC:add Relationships: is a type of regulation of hypersensitivity [GO:0002883]; is a type of regulation of myeloid leukocyte mediated immunity [GO:0002886]; is a type of regulation of immunoglobulin mediated immune response [GO:0002889]; regulates type II hypersensitivity [GO:0002445] Subtypes: GO:0001796, regulation of type IIb hypersensitivity [GO:0001799], negative regulation of type II hypersensitivity [GO:0002893], GO:0002894